{
  "gene": "UniProtKB:Q9NPC3",
  "gene_name": "E3 ubiquitin-protein ligase CCNB1IP1",
  "term_id": "UNKNOWN:0001",
  "term_label": "Unknown molecular function",
  "gene_symbol": "CCNB1IP1"
}